{
  "gene_name": "Protein FAM237A",
  "gene": "UniProtKB:A0A1B0GTK4",
  "term_id": "UNKNOWN:0003",
  "gene_symbol": "FAM237A",
  "term_label": "Unknown cellular component"
}